{
  "term_id": "GO:0071363",
  "gene_symbol": "ACVR2B",
  "term_label": "cellular response to growth factor stimulus",
  "gene_name": "Activin receptor type-2B",
  "gene": "UniProtKB:Q13705"
}